{
  "term_id": "GO:0002230",
  "gene": "UniProtKB:Q8N884",
  "gene_name": "Cyclic GMP-AMP synthase",
  "gene_symbol": "CGAS",
  "term_label": "positive regulation of defense response to virus by host"
}